{
  "gene": "UniProtKB:Q5JRM2",
  "term_id": "UNKNOWN:0003",
  "gene_symbol": "CXorf66",
  "gene_name": "Uncharacterized protein CXorf66",
  "term_label": "Unknown cellular component"
}